positive regulation of antisense RNA transcription [GO:0060196] (biological process) Definition: Any process that increases the frequency, rate or extent of the synthesis of antisense RNA, an RNA molecule complementary in sequence to another RNA or DNA molecule, which, by binding the latter, acts to inhibit its function and/or completion of synthesis, on a template of DNA. Relationships: is a type of positive regulation of DNA-templated transcription [GO:0045893]; is a type of regulation of antisense RNA transcription [GO:0060194]; positively regulates antisense RNA transcription [GO:0009300] References: PMID:18075583 Sources: GOC:dph, GOC:tb